DNA polymerase complex [GO:0042575] (cellular component) Subtypes: alpha DNA polymerase:primase complex [GO:0005658], gamma DNA polymerase complex [GO:0005760], epsilon DNA polymerase complex [GO:0008622], DNA polymerase V complex [GO:0009355], DNA polymerase III complex [GO:0009360], zeta DNA polymerase complex [GO:0016035], delta DNA polymerase complex [GO:0043625] Definition: A protein complex that possesses DNA polymerase activity and is involved in template directed synthesis of DNA. References: PMID:12045093 Sources: GOC:jl Relationships: is_a transferase complex, transferring phosphorus-containing groups [GO:0061695]; is a type of GO:0140535